{
  "gene_name": "Scavenger receptor cysteine-rich type 1 protein M130",
  "term_id": "UNKNOWN:0002",
  "gene": "UniProtKB:Q86VB7",
  "term_label": "Unknown biological process",
  "gene_symbol": "CD163"
}